{
  "term_label": "Unknown molecular function",
  "gene_name": "Coiled-coil domain-containing protein 39",
  "gene": "UniProtKB:Q9UFE4",
  "gene_symbol": "CCDC39",
  "term_id": "UNKNOWN:0001"
}